{
  "term_label": "ERAD pathway",
  "gene_name": "Rhomboid domain-containing protein 2",
  "term_id": "GO:0036503",
  "gene": "UniProtKB:Q6NTF9",
  "gene_symbol": "RHBDD2"
}